{
  "gene": "UniProtKB:Q9Y2B5",
  "term_label": "guanyl-nucleotide exchange factor activity",
  "gene_symbol": "VPS9D1",
  "term_id": "GO:0005085",
  "gene_name": "VPS9 domain-containing protein 1"
}